{
  "gene": "UniProtKB:Q15072",
  "term_id": "GO:0000981",
  "gene_symbol": "ZNF146",
  "gene_name": "Zinc finger protein OZF",
  "term_label": "DNA-binding transcription factor activity, RNA polymerase II-specific"
}